{
  "term_id": "GO:0007186",
  "term_label": "G protein-coupled receptor signaling pathway",
  "gene_name": "Phosphoinositide 3-kinase regulatory subunit 5",
  "gene": "UniProtKB:Q8WYR1",
  "gene_symbol": "PIK3R5"
}